{
  "gene": "UniProtKB:O43660",
  "gene_symbol": "PLRG1",
  "term_label": "catalytic step 2 spliceosome",
  "gene_name": "Pleiotropic regulator 1",
  "term_id": "GO:0071013"
}